{
  "gene_name": "Huntingtin",
  "term_label": "vesicle transport along microtubule",
  "gene_symbol": "HTT",
  "gene": "UniProtKB:P42858",
  "term_id": "GO:0047496"
}